ER to chloroplast lipid transport [GO:1990052] (biological process) References: PMID:18689504 Definition: The directed movement of a lipid from the endoplasmic reticulum (ER) to the chloroplast. Relationships: is a type of intracellular lipid transport [GO:0032365]; is a type of endoplasmic reticulum to chloroplast transport [GO:1901965] Also known as: ER to chloroplast lipid trafficking, endoplasmic reticulum to chloroplast lipid transport